positive regulation of toll-like receptor 5 signaling pathway [GO:0034149] (biological process) Definition: Any process that activates or increases the frequency, rate, or extent of toll-like receptor 5 signaling pathway. References: PMID:16551253, PMID:17328678 Sources: GOC:add Relationships: is a type of regulation of toll-like receptor 5 signaling pathway [GO:0034147]; is a type of positive regulation of pattern recognition receptor signaling pathway [GO:0062208]; positively regulates toll-like receptor 5 signaling pathway [GO:0034146] Also known as: positive regulation of TLR5 signaling pathway, positive regulation of toll-like receptor 5 signalling pathway